{
  "term_label": "signaling receptor binding",
  "gene_name": "Protein BEX5",
  "term_id": "GO:0005102",
  "gene": "UniProtKB:Q5H9J7",
  "gene_symbol": "BEX5"
}